phosphoamidase activity [GO:0050187] (molecular function) Relationships: is_a hydrolase activity, acting on acid phosphorus-nitrogen bonds [GO:0016825] Sources: RHEA:12977 Definition: Catalysis of the reaction: N-phosphocreatine + H2O = creatine + phosphate. Also known as: creatine phosphatase activity, phosphamide hydrolase activity